{
  "term_id": "GO:0008053",
  "term_label": "mitochondrial fusion",
  "gene_name": "Mitoguardin 2",
  "gene": "UniProtKB:Q7L4E1",
  "gene_symbol": "MIGA2"
}